{
  "gene": "UniProtKB:Q2NL82",
  "term_id": "GO:0000479",
  "term_label": "endonucleolytic cleavage of tricistronic rRNA transcript (SSU-rRNA, 5.8S rRNA, LSU-rRNA)",
  "gene_name": "Pre-rRNA-processing protein TSR1 homolog",
  "gene_symbol": "TSR1"
}